{
  "gene_symbol": "RBM5",
  "gene": "UniProtKB:P52756",
  "term_id": "GO:0000398",
  "gene_name": "RNA-binding protein 5",
  "term_label": "mRNA splicing, via spliceosome"
}